{
  "gene_symbol": "KCNE3",
  "gene_name": "Potassium voltage-gated channel subfamily E member 3",
  "term_id": "UNKNOWN:0003",
  "term_label": "Unknown cellular component",
  "gene": "UniProtKB:Q9Y6H6"
}